{
  "term_label": "neuron differentiation",
  "gene": "UniProtKB:P36873",
  "gene_name": "Serine_threonine-protein phosphatase PP1-gamma catalytic subunit",
  "gene_symbol": "PPP1CC",
  "term_id": "GO:0030182"
}